{
  "gene_name": "Pyridoxal-dependent decarboxylase domain-containing protein 1",
  "term_label": "Unknown cellular component",
  "gene_symbol": "PDXDC1",
  "gene": "UniProtKB:Q6P996",
  "term_id": "UNKNOWN:0003"
}